{
  "term_id": "GO:0019901",
  "gene": "UniProtKB:P54829",
  "gene_name": "Tyrosine-protein phosphatase non-receptor type 5",
  "term_label": "protein kinase binding",
  "gene_symbol": "PTPN5"
}